positive regulation of epithelium regeneration [GO:1905043] (biological process) Definition: Any process that activates or increases the frequency, rate or extent of epithelium regeneration. Also known as: positive regulation of regeneration of epithelium, up regulation of epithelium regeneration, up regulation of regeneration of epithelium, up-regulation of epithelium regeneration, up-regulation of regeneration of epithelium, upregulation of epithelium regeneration, upregulation of regeneration of epithelium, activation of epithelium regeneration, activation of regeneration of epithelium References: PMID:23221517 Sources: GOC:BHF, GOC:BHF_miRNA, GOC:TermGenie, GOC:rph, GO_REF:0000058 Relationships: is a type of positive regulation of developmental growth [GO:0048639]; is a type of regulation of epithelium regeneration [GO:1905041]; positively regulates epithelium regeneration [GO:1990399]